maintenance of translational fidelity [GO:1990145] (biological process) References: PMID:21841312 Sources: GOC:hjd, ISBN:9781936113460 Definition: Suppression of the occurrence of translational errors, such as codon-anticodon mis-paring, during the process of translation of a protein using an mRNA template. Relationships: is a type of macromolecule biosynthetic process [GO:0009059]; is part of translation [GO:0006412]